adenine catabolic process [GO:0006146] (biological process) Relationships: is a type of purine nucleobase catabolic process [GO:0006145]; is a type of adenine metabolic process [GO:0046083] Sources: ISBN:0198506732 Also known as: adenine breakdown, adenine catabolism, adenine degradation Definition: The chemical reactions and pathways resulting in the breakdown of adenine, 6-aminopurine, one of the 5 main bases found in nucleic acids and a component of numerous important derivatives of its corresponding ribonucleoside, adenosine.